{
  "gene_symbol": "CCDC190",
  "gene_name": "Coiled-coil domain-containing protein 190",
  "gene": "UniProtKB:Q86UF4",
  "term_label": "Unknown cellular component",
  "term_id": "UNKNOWN:0003"
}